negative regulation of mucus secretion [GO:0070256] (biological process) Also known as: negative regulation of mucus production Definition: Any process that stops, prevents, or reduces the frequency, rate or extent of the regulated release of mucus from a cell or a tissue. Sources: GOC:add Relationships: is a type of negative regulation of secretion [GO:0051048]; is a type of negative regulation of multicellular organismal process [GO:0051241]; is a type of regulation of mucus secretion [GO:0070255]; negatively regulates mucus secretion [GO:0070254]